{
  "gene_symbol": "SPATA31F1",
  "gene": "UniProtKB:Q6ZU69",
  "gene_name": "Protein SPATA31F1",
  "term_label": "Unknown biological process",
  "term_id": "UNKNOWN:0002"
}